{
  "gene_symbol": "TFDP1",
  "term_id": "GO:0006357",
  "gene": "UniProtKB:Q14186",
  "term_label": "regulation of transcription by RNA polymerase II",
  "gene_name": "Transcription factor Dp-1"
}